{
  "gene_name": "Small ribosomal subunit protein eS7",
  "term_id": "GO:0003735",
  "gene_symbol": "RPS7",
  "term_label": "structural constituent of ribosome",
  "gene": "UniProtKB:P62081"
}